{
  "gene_name": "Steroid receptor-associated and regulated protein",
  "gene": "UniProtKB:Q8NEQ6",
  "term_id": "GO:0005737",
  "term_label": "cytoplasm",
  "gene_symbol": "SRARP"
}